protein phosphatase inhibitor activity [GO:0004864] (molecular function) Subtypes: protein serine/threonine phosphatase inhibitor activity [GO:0004865] Definition: Binds to and stops, prevents or reduces the activity of a protein phosphatase. Relationships: is a type of GO:0019212; is a type of protein phosphatase regulator activity [GO:0019888]; negatively regulates phosphoprotein phosphatase activity [GO:0004721] Also known as: phosphoprotein phosphatase inhibitor activity, protein phosphatase 2 inhibitor activity, protein phosphatase type 2A inhibitor activity Sources: GOC:ai